{
  "gene": "UniProtKB:P63208",
  "term_label": "nucleus",
  "term_id": "GO:0005634",
  "gene_symbol": "SKP1",
  "gene_name": "S-phase kinase-associated protein 1"
}